rhabdomere morphogenesis [GO:0061541] (biological process) References: PMID:22113834 Sources: GOC:dph Definition: The process in which the anatomical structures of a rhabdomere are generated and organized. The rhabdomere is the organelle on the apical surface of a photoreceptor cell that contains the visual pigments. Relationships: is a type of neuron projection morphogenesis [GO:0048812]; is part of photoreceptor cell morphogenesis [GO:0008594]; is part of rhabdomere development [GO:0042052]